{
  "gene": "UniProtKB:Q9ULW8",
  "term_id": "GO:0004668",
  "term_label": "protein-arginine deiminase activity",
  "gene_symbol": "PADI3",
  "gene_name": "Protein-arginine deiminase type-3"
}